sperm fibrous sheath [GO:0035686] (cellular component) Definition: A cytoskeletal structure surrounding the axoneme and outer dense fibers of the sperm flagellum. Consists of two longitudinal columns connected by closely arrayed semicircular ribs that assemble from distal to proximal throughout spermiogenesis. The fibrous sheath probably influences the degree of flexibility, plane of flagellar motion, and the shape of the flagellar beat. Relationships: is a type of GO:0110165; is part of sperm flagellum [GO:0036126] Also known as: flagellar fibrous sheath, flagellum fibrous sheath References: PMID:20731842, PMID:3282552 Sources: GOC:BHF, GOC:cilia, GOC:krc